{
  "term_id": "UNKNOWN:0003",
  "gene_name": "Max-interacting protein 1",
  "gene_symbol": "MXI1",
  "gene": "UniProtKB:P50539",
  "term_label": "Unknown cellular component"
}